protein storage vacuole [GO:0000326] (cellular component) Relationships: is a type of storage vacuole [GO:0000322]; is_a GO:0000325 Definition: A storage vacuole that contains a lytic vacuole; identified in plants. References: PMID:11739409